{
  "gene_symbol": "NKX2-8",
  "term_id": "GO:0000981",
  "gene": "UniProtKB:O15522",
  "term_label": "DNA-binding transcription factor activity, RNA polymerase II-specific",
  "gene_name": "Homeobox protein Nkx-2.8"
}